{
  "gene_symbol": "TPRG1L",
  "gene_name": "Tumor protein p63-regulated gene 1-like protein",
  "term_id": "UNKNOWN:0002",
  "gene": "UniProtKB:Q5T0D9",
  "term_label": "Unknown biological process"
}